galactinol-raffinose galactosyltransferase activity [GO:0047268] (molecular function) Definition: Catalysis of the reaction: raffinose + 1-alpha-D-galactosyl-myo-inositol = stachyose + myo-inositol. Relationships: is a type of galactosyltransferase activity [GO:0008378] Also known as: alpha-D-(1->3)-galactosyl-myo-inositol:raffinose galactosyltransferase activity, stachyose synthetase activity Sources: EC:2.4.1.67, MetaCyc:2.4.1.67-RXN